alkylbase DNA N-glycosylase activity [GO:0003905] (molecular function) References: PMID:10872450, PMID:9224623 Sources: EC:3.2.2.21, GOC:elh Also known as: alkylated-DNA glycohydrolase (releasing methyladenine and methylguanine), DNA-3-methyladenine glycosidase II activity, alkylbase DNA glycosidase activity, 3-methyladenine DNA glycosylase II, AlkA, DNA glycosidase II activity, DNA-3-methyladenine glycosylase II, deoxyribonucleate 3-methyladenine glycosidase II Definition: Catalysis of the reaction: DNA with alkylated base + H2O = DNA with abasic site + alkylated base. This reaction is the hydrolysis of DNA by cleavage of the N-C1' glycosidic bond between the target damaged DNA base and the deoxyribose sugar to remove an alkylated base, leaving an apyrimidinic or apurinic site. Subtypes: GO:0043733, GO:0043916, DNA-1,N6-ethenoadenine N-glycosylase activity [GO:0052820], DNA-7-methyladenine glycosylase activity [GO:0052821], GO:1990053 Relationships: is a type of GO:0019104